cyclodextrin binding [GO:2001073] (molecular function) Relationships: is a type of polysaccharide binding [GO:0030247]; is a type of oligosaccharide binding [GO:0070492] Definition: Binding to cyclodextrin. Sources: GOC:mengo_curators